{
  "gene": "UniProtKB:Q96J84",
  "term_label": "plasma membrane",
  "term_id": "GO:0005886",
  "gene_name": "Kin of IRRE-like protein 1",
  "gene_symbol": "KIRREL1"
}